{
  "term_id": "GO:0006355",
  "gene_symbol": "ZNF253",
  "gene_name": "Zinc finger protein 253",
  "term_label": "regulation of DNA-templated transcription",
  "gene": "UniProtKB:O75346"
}